2-aminoethylphosphonate-pyruvate transaminase activity [GO:0047304] (molecular function) Also known as: 2-aminoethylphosphonate-pyruvate aminotransferase activity, (2-aminoethyl)phosphonate aminotransferase activity, (2-aminoethyl)phosphonate transaminase activity, (2-aminoethyl)phosphonate--pyruvate aminotransferase activity, (2-aminoethyl)phosphonate:pyruvate aminotransferase activity, (2-aminoethyl)phosphonic acid aminotransferase activity, 2-aminoethylphosphonate aminotransferase activity, 2-aminoethylphosphonate--pyruvate aminotransferase activity Sources: EC:2.6.1.37, RHEA:17021 Definition: Catalysis of the reaction: (2-aminoethyl)phosphonate + pyruvate = L-alanine + phosphonoacetaldehyde. Relationships: is a type of GO:0008483